{
  "gene_symbol": "LCMT1",
  "term_label": "protein C-terminal leucine carboxyl O-methyltransferase activity",
  "gene_name": "Leucine carboxyl methyltransferase 1",
  "gene": "UniProtKB:Q9UIC8",
  "term_id": "GO:0018423"
}